{
  "gene_name": "Collagen alpha-4(IV) chain",
  "gene": "UniProtKB:P53420",
  "term_id": "GO:0005587",
  "gene_symbol": "COL4A4",
  "term_label": "collagen type IV trimer"
}